vagus nerve formation [GO:0021646] (biological process) Relationships: is a type of cranial nerve formation [GO:0021603]; is part of GO:0021644 Definition: The process that gives rise to the vagus nerve. This process pertains to the initial formation of a structure from unspecified parts. This nerve is primarily sensory but also has visceromotor components. It originates in the brain stem and controls many autonomic functions of the heart, lungs, stomach, pharynx, larynx, trachea, esophagus and other gastrointestinal tract components. It controls some motor functions such as speech. The sensory branches mediate sensation from the pharynx, larynx, thorax and abdomen; it also innervates taste buds in the epiglottis. Sources: GOC:cls, GOC:dgh, GOC:dph, GOC:jid, GO_REF:0000021 Also known as: CN X biosynthesis, CN X formation